regulation of protein targeting to vacuole involved in autophagy [GO:1904051] (biological process) Definition: Any process that modulates the frequency, rate or extent of protein targeting to vacuole involved in autophagy. References: PMID:22020285 Sources: GOC:PARL, GOC:TermGenie, GOC:pad, GO_REF:0000058 Relationships: is a type of regulation of intracellular protein transport [GO:0033157]; is a type of regulation of vacuolar transport [GO:1903335]; is a type of GO:1903533; regulates protein targeting to vacuole involved in autophagy [GO:0071211] Note: An example of this is SMURF1 in human (UniProt symbol Q9HCE7) in PMID:22020285 (inferred from mutant phenotype). Subtypes: negative regulation of protein targeting to vacuole involved in autophagy [GO:1904052], positive regulation of protein targeting to vacuole involved in autophagy [GO:1904053]